{
  "gene": "UniProtKB:Q13275",
  "term_label": "neural crest cell migration",
  "gene_symbol": "SEMA3F",
  "term_id": "GO:0001755",
  "gene_name": "Semaphorin-3F"
}